{
  "term_id": "GO:0004984",
  "gene_symbol": "OR2T4",
  "term_label": "olfactory receptor activity",
  "gene_name": "Olfactory receptor 2T4",
  "gene": "UniProtKB:Q8NH00"
}